{
  "term_label": "olfactory receptor activity",
  "term_id": "GO:0004984",
  "gene_name": "Olfactory receptor 10K2",
  "gene": "UniProtKB:Q6IF99",
  "gene_symbol": "OR10K2"
}